fumiquinazoline C biosynthetic process [GO:1900781] (biological process) Relationships: is a type of indole alkaloid biosynthetic process [GO:0035835] Definition: The chemical reactions and pathways resulting in the formation of the indole alkaloid fumiquinazoline C. References: PMID:20225828 Sources: GOC:TermGenie, GOC:di Also known as: fumiquinazoline C metabolic process, fumiquinazoline C metabolism, fumiquinazoline biosynthetic process, fumiquinazoline metabolic process, fumiquinazoline metabolism, fumiquinazoline C anabolism, fumiquinazoline C biosynthesis, fumiquinazoline C formation, fumiquinazoline C synthesis, fumiquinazoline biosynthesis, fumiquinazolines synthesis